{
  "gene_symbol": "UFSP2",
  "gene_name": "Ufm1-specific protease 2",
  "gene": "UniProtKB:Q9NUQ7",
  "term_label": "deUFMylase activity",
  "term_id": "GO:0071567"
}